{
  "gene": "UniProtKB:O15523",
  "term_label": "P granule",
  "term_id": "GO:0043186",
  "gene_name": "ATP-dependent RNA helicase DDX3Y",
  "gene_symbol": "DDX3Y"
}